cytoskeleton of presynaptic active zone [GO:0048788] (cellular component) References: PMID:10944438 Sources: GOC:dh, GOC:dl, GOC:ef, GOC:jid, NIF_Subcellular:sao1470121605 Also known as: active zone cytomatrix, pre-synaptic cytoskeletal matrix assembled at active zones, presynaptic cytomatrix assembled at active zones, presynaptic cytoskeletal matrix, presynaptic cytoskeletal matrix assembled at active zones, CAZ, T-bar, T-bar ribbon, pre-synaptic dense body, presynaptic dense body, synaptic ribbon, pre-synaptic ribbon, presynaptic ribbon, ribbon Subtypes: GO:0098980 Relationships: is a type of GO:0030863; is_a presynaptic cytoskeleton [GO:0099569]; is part of presynaptic active zone cytoplasmic component [GO:0098831] Definition: The specialized cytoskeletal matrix of the presynaptic active zone. It has specialized functions in organizing synaptic events such as immobilisation or translocation of synaptic vesicles, and assembling active zone components. It is believed to form a molecular scaffold that organizes neurotransmitter release sites.